{
  "term_id": "GO:0045499",
  "term_label": "chemorepellent activity",
  "gene": "UniProtKB:Q9P283",
  "gene_name": "Semaphorin-5B",
  "gene_symbol": "SEMA5B"
}